{
  "term_id": "GO:0005085",
  "term_label": "guanyl-nucleotide exchange factor activity",
  "gene_name": "Guanine nucleotide exchange factor for Rab-3A",
  "gene": "UniProtKB:Q8TBN0",
  "gene_symbol": "RAB3IL1"
}